{
  "gene": "UniProtKB:P28330",
  "term_id": "GO:0033539",
  "term_label": "fatty acid beta-oxidation using acyl-CoA dehydrogenase",
  "gene_name": "Long-chain specific acyl-CoA dehydrogenase, mitochondrial",
  "gene_symbol": "ACADL"
}